regulation of defense response to bacterium [GO:1900424] (BP) Relationships: is a type of regulation of response to biotic stimulus [GO:0002831]; is a type of regulation of defense response [GO:0031347]; is a type of regulation of response to external stimulus [GO:0032101]; regulates defense response to bacterium [GO:0042742] Definition: Any process that modulates the frequency, rate or extent of defense response to bacterium. Also known as: regulation of defence response to bacteria, regulation of defence response to bacterium, regulation of defense response to bacteria, regulation of defence response to bacterium, incompatible interaction, regulation of defence response to pathogenic bacteria, incompatible interaction, regulation of defence response to pathogenic bacterium, incompatible interaction, regulation of defense response to bacterium, incompatible interaction, regulation of resistance response to pathogenic bacteria, regulation of resistance response to pathogenic bacterium, regulation of antibacterial peptide activity Subtypes: negative regulation of defense response to bacterium [GO:1900425], GO:1900426 References: PMID:22346749 Sources: GOC:TermGenie